positive regulation of methanophenazine biosynthetic process [GO:1900964] (biological process) Relationships: is a type of positive regulation of biosynthetic process [GO:0009891]; is a type of GO:1900962; positively regulates methanophenazine biosynthetic process [GO:1900630] Also known as: activation of methanophenazine anabolism, activation of methanophenazine biosynthesis, activation of methanophenazine formation, activation of methanophenazine synthesis, positive regulation of methanophenazine anabolism, positive regulation of methanophenazine biosynthesis, positive regulation of methanophenazine formation, positive regulation of methanophenazine synthesis, up regulation of methanophenazine anabolism, up regulation of methanophenazine biosynthesis, up regulation of methanophenazine biosynthetic process, up regulation of methanophenazine formation, up regulation of methanophenazine synthesis, up-regulation of methanophenazine anabolism, up-regulation of methanophenazine biosynthesis, up-regulation of methanophenazine biosynthetic process, up-regulation of methanophenazine formation, up-regulation of methanophenazine synthesis, upregulation of methanophenazine anabolism, upregulation of methanophenazine biosynthesis, upregulation of methanophenazine biosynthetic process, upregulation of methanophenazine formation, upregulation of methanophenazine synthesis, activation of methanophenazine biosynthetic process Sources: GOC:TermGenie, GOC:mengo_curators Definition: Any process that activates or increases the frequency, rate or extent of methanophenazine biosynthetic process.